{
  "term_label": "Unknown molecular function",
  "gene_symbol": "TTR",
  "gene": "UniProtKB:P02766",
  "gene_name": "Transthyretin",
  "term_id": "UNKNOWN:0001"
}